positive regulation of exit from meiosis [GO:0106062] (biological process) Relationships: is a type of regulation of exit from meiosis [GO:0106060]; is a type of positive regulation of meiotic cell cycle phase transition [GO:1901995]; positively regulates exit from meiosis [GO:1990947] References: PMID:11493649 Sources: GOC:al Definition: Any process that activates or increases the frequency, rate or extent of exit from meiosis.